{
  "gene_name": "Transcription elongation factor A protein 3",
  "gene": "UniProtKB:O75764",
  "gene_symbol": "TCEA3",
  "term_label": "transcription elongation by RNA polymerase II",
  "term_id": "GO:0006368"
}